{
  "gene_name": "Uncharacterized protein CXorf49",
  "term_label": "Unknown biological process",
  "term_id": "UNKNOWN:0002",
  "gene": "UniProtKB:A8MYA2",
  "gene_symbol": "CXorf49B"
}